{
  "gene": "UniProtKB:Q9C002",
  "term_label": "Unknown biological process",
  "gene_symbol": "NMES1",
  "term_id": "UNKNOWN:0002",
  "gene_name": "Normal mucosa of esophagus-specific gene 1 protein"
}